{
  "gene": "UniProtKB:A8MTB9",
  "gene_name": "Carcinoembryonic antigen-related cell adhesion molecule 18",
  "term_label": "heterophilic cell-cell adhesion",
  "term_id": "GO:0007157",
  "gene_symbol": "CEACAM18"
}